Gin4 complex [GO:1990317] (cellular component) Relationships: is a type of serine/threonine protein kinase complex [GO:1902554]; is part of cellular bud neck septin ring [GO:0000144] Also known as: Gin4-septin complex References: PMID:12058072 Sources: GOC:bhm Definition: A protein complex involved in septin ring formation during mitosis. In Saccharomyces cerevisiae it consists of BNI5, CDC3, CDC10, CDC11, CDC12, GIN4, NAP1 and SHS1. At least 2 GIN4 molecules are involved.